{
  "gene": "UniProtKB:Q9Y239",
  "term_label": "pattern recognition receptor signaling pathway",
  "term_id": "GO:0002221",
  "gene_symbol": "NOD1",
  "gene_name": "Nucleotide-binding oligomerization domain-containing protein 1"
}